oxalate biosynthetic process [GO:0033610] (biological process) Relationships: is a type of GO:0033609; is a type of GO:0043650 Definition: The chemical reactions and pathways resulting in the formation of oxalate, the organic acid ethanedioate. Sources: GOC:mlg Also known as: ethanedioate biosynthetic process, ethanedioic acid biosynthetic process, oxalate anabolism, oxalate biosynthesis, oxalate formation, oxalate synthesis, oxalic acid biosynthetic process